{
  "gene_symbol": "SOX15",
  "gene": "UniProtKB:O60248",
  "term_id": "GO:0007420",
  "term_label": "brain development",
  "gene_name": "Protein SOX-15"
}